{
  "gene": "UniProtKB:P0DTW1",
  "gene_name": "G antigen 1",
  "term_id": "UNKNOWN:0001",
  "gene_symbol": "GAGE1",
  "term_label": "Unknown molecular function"
}